{
  "gene_name": "Bifunctional heparan sulfate N-deacetylase_N-sulfotransferase 2",
  "term_label": "heparan sulfate N-sulfotransferase activity",
  "gene": "UniProtKB:P52849",
  "gene_symbol": "NDST2",
  "term_id": "GO:0015016"
}